{
  "term_id": "GO:0033152",
  "gene": "UniProtKB:P15923",
  "term_label": "immunoglobulin V(D)J recombination",
  "gene_symbol": "TCF3",
  "gene_name": "Transcription factor E2-alpha"
}